{
  "gene": "UniProtKB:Q3KNS6",
  "gene_name": "Zinc finger protein 829",
  "term_id": "GO:0000981",
  "term_label": "DNA-binding transcription factor activity, RNA polymerase II-specific",
  "gene_symbol": "ZNF829"
}